{
  "term_label": "Unknown biological process",
  "gene": "UniProtKB:O95500",
  "gene_symbol": "CLDN14",
  "term_id": "UNKNOWN:0002",
  "gene_name": "Claudin-14"
}